negative regulation of termination of RNA polymerase II transcription [GO:0120191] (biological process) References: PMID:29899453 Sources: GOC:krc, GOC:vw Subtypes: negative regulation of termination of RNA polymerase II transcription, poly(A)-coupled [GO:2000805] Relationships: is a type of negative regulation of transcription by RNA polymerase II [GO:0000122]; is a type of negative regulation of termination of DNA-templated transcription [GO:0060567]; is a type of GO:1904594; negatively regulates termination of RNA polymerase II transcription [GO:0006369] Also known as: down regulation of RNA 3'-end formation by RNA polymerase II, down regulation of RNA polymerase II transcription termination, down regulation of termination of RNA polymerase II transcription, down regulation of transcription termination from Pol II promoter, down regulation of transcription termination from RNA polymerase II promoter, down-regulation of RNA 3'-end formation by RNA polymerase II, down-regulation of RNA polymerase II transcription termination, down-regulation of termination of RNA polymerase II transcription, down-regulation of transcription termination from Pol II promoter, down-regulation of transcription termination from RNA polymerase II promoter, downregulation of RNA 3'-end formation by RNA polymerase II, downregulation of RNA polymerase II transcription termination, downregulation of termination of RNA polymerase II transcription, downregulation of transcription termination from Pol II promoter, downregulation of transcription termination from RNA polymerase II promoter, negative regulation of RNA 3'-end formation by RNA polymerase II, negative regulation of RNA polymerase II transcription termination, negative regulation of transcription termination from Pol II promoter, negative regulation of transcription termination from RNA polymerase II promoter, repression of RNA 3'-end formation by RNA polymerase II, repression of RNA polymerase II transcription termination, repression of termination of RNA polymerase II transcription, repression of transcription termination from Pol II promoter, repression of transcription termination from RNA polymerase II promoter, down regulation of RNA polymerase II transcription termination factor activity, down-regulation of RNA polymerase II transcription termination factor activity, downregulation of RNA polymerase II transcription termination factor activity, negative regulation of RNA polymerase II transcription termination factor activity, repression of RNA polymerase II transcription termination factor activity Definition: Any process that stops, prevents or reduces the frequency, rate or extent of termination of RNA polymerase II transcription.